{
  "gene_name": "Uncharacterized protein",
  "gene_symbol": "A0A494C176",
  "term_label": "Unknown cellular component",
  "term_id": "UNKNOWN:0003",
  "gene": "UniProtKB:A0A494C176"
}